mitotic sister chromatid biorientation [GO:1990758] (BP) Definition: The mitotic cell cycle process in which sister chromatids establish stable, end-on attachments to the plus ends of microtubules emanating from opposite spindle poles, oriented such that separation can proceed. This is the final step in metaphase plate congression. References: PMID:15309047, PMID:26258632, PMID:26705896 Relationships: is a type of sister chromatid biorientation [GO:0031134]; is a type of attachment of mitotic spindle microtubules to kinetochore [GO:0051315]; has part microtubule plus-end binding [GO:0051010] Regulation: RO_0002213 by GO:0140429